{
  "gene_name": "RNA guanine-N7 methyltransferase activating subunit",
  "gene": "UniProtKB:Q9BTL3",
  "gene_symbol": "RAMAC",
  "term_label": "RNA binding",
  "term_id": "GO:0003723"
}